{
  "gene_name": "Trafficking protein particle complex subunit 3-like protein",
  "gene_symbol": "TRAPPC3L",
  "gene": "UniProtKB:Q5T215",
  "term_label": "guanyl-nucleotide exchange factor activity",
  "term_id": "GO:0005085"
}